{
  "gene_symbol": "ZMYM6",
  "gene": "UniProtKB:O95789",
  "term_label": "Unknown cellular component",
  "gene_name": "Zinc finger MYM-type protein 6",
  "term_id": "UNKNOWN:0003"
}